{
  "gene_name": "Uncharacterized protein",
  "term_id": "UNKNOWN:0002",
  "term_label": "Unknown biological process",
  "gene": "UniProtKB:A0A8V8TLL3",
  "gene_symbol": "A0A8V8TLL3"
}